regulation of protein targeting to mitochondrion [GO:1903214] (BP) Definition: Any process that modulates the frequency, rate or extent of protein targeting to mitochondrion. Sources: GOC:PARL, GOC:TermGenie, GOC:bf, GO_REF:0000058 Also known as: regulation of protein import into mitochondrion, regulation of protein targeting to mitochondria, regulation of protein-mitochondrial targeting, regulation of mitochondrial protein import, regulation of mitochondrial translocation Relationships: is a type of regulation of protein targeting [GO:1903533]; is a type of regulation of establishment of protein localization to mitochondrion [GO:1903747]; regulates GO:0006626 Subtypes: negative regulation of protein targeting to mitochondrion [GO:1903215], regulation of protein insertion into mitochondrial outer membrane [GO:1903636], positive regulation of protein targeting to mitochondrion [GO:1903955]